regulation of mesenchymal stem cell proliferation [GO:1902460] (biological process) Also known as: regulation of MSC proliferation Subtypes: regulation of mesenchymal stem cell proliferation involved in nephron morphogenesis [GO:0072042], negative regulation of mesenchymal stem cell proliferation [GO:1902461], positive regulation of mesenchymal stem cell proliferation [GO:1902462] Definition: Any process that modulates the frequency, rate or extent of mesenchymal stem cell proliferation. Relationships: is a type of regulation of stem cell proliferation [GO:0072091]; regulates GO:0097168 References: PMID:18672106 Sources: GOC:TermGenie, GOC:pm